{
  "term_id": "GO:0019373",
  "gene_symbol": "CYP2B6",
  "gene": "UniProtKB:P20813",
  "term_label": "epoxygenase P450 pathway",
  "gene_name": "Cytochrome P450 2B6"
}